{
  "term_label": "Unknown cellular component",
  "gene_name": "Probable E3 ubiquitin-protein ligase HERC1",
  "gene_symbol": "HERC1",
  "gene": "UniProtKB:Q15751",
  "term_id": "UNKNOWN:0003"
}